{
  "gene_name": "Polyunsaturated fatty acid 5-lipoxygenase",
  "gene_symbol": "ALOX5",
  "gene": "UniProtKB:P09917",
  "term_id": "GO:0005635",
  "term_label": "nuclear envelope"
}